{
  "term_id": "GO:0005737",
  "gene_name": "Dynamin-2",
  "gene_symbol": "DNM2",
  "term_label": "cytoplasm",
  "gene": "UniProtKB:P50570"
}